negative regulation of eclosion [GO:0045804] (biological process) Also known as: down regulation of eclosion, down-regulation of eclosion, downregulation of eclosion, inhibition of eclosion Relationships: is a type of regulation of eclosion [GO:0007563]; is a type of negative regulation of developmental process [GO:0051093]; is_a negative regulation of multicellular organismal process [GO:0051241]; RO_0002212 eclosion [GO:0007562] Definition: Any process that stops, prevents, or reduces the frequency, rate or extent of eclosion. Sources: GOC:go_curators